{
  "term_id": "GO:0006898",
  "gene": "UniProtKB:P22897",
  "gene_symbol": "MRC1",
  "term_label": "receptor-mediated endocytosis",
  "gene_name": "Macrophage mannose receptor 1"
}